{
  "term_id": "GO:0005615",
  "gene_name": "Protein Wnt-9b",
  "term_label": "extracellular space",
  "gene_symbol": "WNT9B",
  "gene": "UniProtKB:O14905"
}